{
  "gene_name": "Fibroblast growth factor receptor 2",
  "gene": "UniProtKB:P21802",
  "term_label": "fibroblast growth factor receptor activity",
  "term_id": "GO:0005007",
  "gene_symbol": "FGFR2"
}